{
  "gene_name": "Protein Wiz",
  "term_label": "nucleus",
  "gene": "UniProtKB:O95785",
  "term_id": "GO:0005634",
  "gene_symbol": "WIZ"
}